{
  "gene_name": "DNA dC-dU-editing enzyme APOBEC-3C",
  "term_label": "P-body",
  "gene_symbol": "APOBEC3C",
  "term_id": "GO:0000932",
  "gene": "UniProtKB:Q9NRW3"
}